division septum assembly [GO:0000917] (biological process) Definition: The assembly and arrangement of a septum that spans the plasma membrane interface between progeny cells following cytokinesis. The progeny cells that form a division septum are not able to exchange intracellular material. Sources: GOC:mtg_cell_cycle Also known as: septation, division septum formation, formation of division septum, division septum assembly involved in cell cycle cytokinesis, division septum assembly involved in cell cycle cytokinesis involved in mitotic cell cycle, division septum formation involved in cell cycle cytokinesis, division septum formation involved in cell cycle cytokinesis involved in mitotic cell cycle, division septum formation involved in mitotic cell cycle, formation of division septum involved in mitotic cell cycle, mitotic division septum assembly, septin assembly and septum biosynthesis involved in mitotic cell cycle, septin assembly and septum formation involved in mitotic cell cycle, septin assembly and septum biosynthesis, septin assembly and septum formation Relationships: is a type of cell septum assembly [GO:0090529] Subtypes: mitotic division septum assembly [GO:0140278] Regulation: RO_0002213 by GO:0010973; RO_0002212 by negative regulation of division septum assembly [GO:0010974]; regulated by regulation of division septum assembly [GO:0032955]